{
  "term_label": "Unknown biological process",
  "gene_name": "Inter-alpha-trypsin inhibitor heavy chain H4",
  "gene": "UniProtKB:Q14624",
  "term_id": "UNKNOWN:0002",
  "gene_symbol": "ITIH4"
}